{
  "term_id": "GO:0016477",
  "gene_symbol": "CDH3",
  "gene_name": "Cadherin-3",
  "gene": "UniProtKB:P22223",
  "term_label": "cell migration"
}